{
  "gene_symbol": "SNX33",
  "gene": "UniProtKB:Q8WV41",
  "gene_name": "Sorting nexin-33",
  "term_label": "endocytosis",
  "term_id": "GO:0006897"
}